cell proliferation in midbrain [GO:0033278] (biological process) Relationships: is a type of neural precursor cell proliferation [GO:0061351]; is part of midbrain development [GO:0030901] Sources: GOC:dgf, GO_REF:0000021 Regulation: RO_0002211 by regulation of cell proliferation in midbrain [GO:1904933]; RO_0002212 by negative regulation of cell proliferation in midbrain [GO:1904934]; positively regulated by positive regulation of cell proliferation in midbrain [GO:1904935] Also known as: cell proliferation in mesencephalon, mesencepahalic cell proliferation Definition: The multiplication or reproduction of cells, resulting in the expansion of a cell population in the midbrain.